{
  "gene_symbol": "ROBO4",
  "gene_name": "Roundabout homolog 4",
  "term_label": "dendrite self-avoidance",
  "term_id": "GO:0070593",
  "gene": "UniProtKB:Q8WZ75"
}